{
  "term_id": "GO:0043410",
  "gene": "UniProtKB:P31371",
  "gene_symbol": "FGF9",
  "term_label": "positive regulation of MAPK cascade",
  "gene_name": "Fibroblast growth factor 9"
}